{
  "term_id": "GO:0000281",
  "gene_symbol": "ANLN",
  "term_label": "mitotic cytokinesis",
  "gene": "UniProtKB:Q9NQW6",
  "gene_name": "Anillin"
}